{
  "gene_symbol": "TRIM51",
  "gene_name": "Tripartite motif-containing protein 51",
  "term_id": "GO:0010468",
  "gene": "UniProtKB:Q9BSJ1",
  "term_label": "regulation of gene expression"
}